{
  "gene": "UniProtKB:Q14164",
  "gene_name": "Inhibitor of nuclear factor kappa-B kinase subunit epsilon",
  "term_label": "cytoplasm",
  "gene_symbol": "IKBKE",
  "term_id": "GO:0005737"
}